{
  "gene_name": "Soluble scavenger receptor cysteine-rich domain-containing protein SSC5D",
  "gene": "UniProtKB:A1L4H1",
  "term_id": "GO:0042494",
  "term_label": "detection of bacterial lipoprotein",
  "gene_symbol": "SSC5D"
}